{
  "gene": "UniProtKB:Q96L03",
  "gene_symbol": "SPATA17",
  "term_label": "Unknown cellular component",
  "gene_name": "Spermatogenesis-associated protein 17",
  "term_id": "UNKNOWN:0003"
}